{
  "gene_symbol": "C5orf22",
  "term_id": "UNKNOWN:0001",
  "gene_name": "UPF0489 protein C5orf22",
  "gene": "UniProtKB:Q49AR2",
  "term_label": "Unknown molecular function"
}